{
  "term_label": "nervous system development",
  "gene_name": "Protein inturned",
  "gene_symbol": "INTU",
  "gene": "UniProtKB:Q9ULD6",
  "term_id": "GO:0007399"
}